phosphatidylglycerol acyl-chain remodeling [GO:0036148] (BP) Relationships: is_a phosphatidylglycerol metabolic process [GO:0046471] Definition: Remodeling the acyl chains of phosphatidylglycerol, through sequential deacylation and re-acylation reactions, to generate phosphatidylglycerol containing different types of fatty acid acyl chains. Also known as: phosphatidylglycerol acyl-chain remodelling References: PMID:15485873, PMID:18458083 Sources: GOC:mw